anthranilate metabolic process [GO:0043420] (biological process) Subtypes: GO:0018870, anthranilate catabolic process [GO:0043421] Relationships: is a type of aromatic amino acid metabolic process [GO:0009072]; is a type of monocarboxylic acid metabolic process [GO:0032787]; is a type of benzene-containing compound metabolic process [GO:0042537] Definition: The chemical reactions and pathways involving anthranilate (2-aminobenzoate). Also known as: 2-aminobenzoate metabolic process, 2-aminobenzoate metabolism, anthranilate metabolism, anthranilic acid metabolic process, anthranilic acid metabolism, ortho-aminobenzoic acid metabolic process, ortho-aminobenzoic acid metabolism Sources: GOC:jl